{
  "term_label": "central nervous system development",
  "gene": "UniProtKB:Q04741",
  "gene_name": "Homeobox protein EMX1",
  "gene_symbol": "EMX1",
  "term_id": "GO:0007417"
}